regulation of T cell migration [GO:2000404] (biological process) Subtypes: regulation of T cell chemotaxis [GO:0010819], GO:2000405, GO:2000406, regulation of T cell extravasation [GO:2000407], GO:2000410 Also known as: regulation of T lymphocyte migration, regulation of T-cell migration, regulation of T-lymphocyte migration Sources: GOC:mah Definition: Any process that modulates the frequency, rate or extent of T cell migration. Relationships: is a type of GO:2000401; regulates GO:0072678